positive regulation of protein lipidation [GO:1903061] (biological process) References: PMID:21909394 Sources: GOC:TermGenie, GOC:rph, GO_REF:0000058 Relationships: is a type of positive regulation of protein modification process [GO:0031401]; is a type of positive regulation of lipoprotein metabolic process [GO:0050747]; is a type of regulation of protein lipidation [GO:1903059]; positively regulates protein lipidation [GO:0006497] Definition: Any process that activates or increases the frequency, rate or extent of protein lipidation. Subtypes: positive regulation of peptidyl-L-cysteine S-palmitoylation [GO:1902664] Also known as: positive regulation of lipid:protein modification, positive regulation of protein amino acid lipidation, up regulation of lipid:protein modification, up regulation of protein amino acid lipidation, up regulation of protein lipidation, up-regulation of lipid:protein modification, up-regulation of protein amino acid lipidation, up-regulation of protein lipidation, upregulation of lipid:protein modification, upregulation of protein amino acid lipidation, upregulation of protein lipidation, activation of lipid:protein modification, activation of protein amino acid lipidation, activation of protein lipidation